{
  "gene_name": "Pre-mRNA-processing factor 19",
  "term_id": "GO:0005737",
  "gene": "UniProtKB:Q9UMS4",
  "gene_symbol": "PRPF19",
  "term_label": "cytoplasm"
}